negative regulation of metanephros development [GO:0072217] (biological process) Relationships: is a type of GO:0072215; is a type of negative regulation of kidney development [GO:0090185]; negatively regulates metanephros development [GO:0001656] Definition: Any process that decreases the rate, frequency or extent of metanephros development. Metanephros development is the process whose specific outcome is the progression of the metanephros over time, from its formation to the mature structure. The metanephros is an organ that filters the blood and excretes the end products of body metabolism in the form of urine. Sources: GOC:mtg_kidney_jan10 Subtypes: negative regulation of metanephric glomerulus development [GO:0072299], GO:2000590